cyanelle thylakoid [GO:0009843] (CC) Definition: A thylakoid found in a cyanelle, which is a type of plastid found in certain algae. The cyanelle contains a photosynthetic membrane resembling that of cyanobacteria. Relationships: is a type of GO:0031976; is part of cyanelle [GO:0009842] Sources: GOC:lr, GOC:mah, GOC:mtg_sensu